{
  "term_id": "GO:0097367",
  "gene": "UniProtKB:Q15485",
  "term_label": "carbohydrate derivative binding",
  "gene_name": "Ficolin-2",
  "gene_symbol": "FCN2"
}